{
  "gene_symbol": "CUL4A",
  "term_label": "protein ubiquitination",
  "gene_name": "Cullin-4A",
  "gene": "UniProtKB:Q13619",
  "term_id": "GO:0016567"
}